{
  "gene_symbol": "TSNARE1",
  "term_id": "GO:0048278",
  "gene_name": "t-SNARE domain-containing protein 1",
  "gene": "UniProtKB:Q96NA8",
  "term_label": "vesicle docking"
}